carboxylic ester hydrolase activity [GO:0052689] (molecular function) Subtypes: GO:0002161, 1-alkyl-2-acetylglycerophosphocholine esterase activity [GO:0003847], GO:0004045, arylesterase activity [GO:0004064], cholinesterase activity [GO:0004104], gluconolactonase activity [GO:0004341], juvenile-hormone esterase activity [GO:0004453], phospholipase A2 activity [GO:0004623], sterol ester esterase activity [GO:0004771], triacylglycerol lipase activity [GO:0004806], GO:0008806, phospholipase A1 activity [GO:0008970], 6-phosphogluconolactonase activity [GO:0017057], fatty-acyl-ethyl-ester synthase activity [GO:0030339], GO:0030599, feruloyl esterase activity [GO:0030600], acetylajmaline esterase activity [GO:0033879], short-chain carboxylesterase activity [GO:0034338], L-ascorbate 6-phosphate lactonase activity [GO:0035460], GO:0035560, GO:0043905, Ser(Gly)-tRNA(Ala) hydrolase activity [GO:0043908], acetylxylan esterase activity [GO:0046555], lactonohydrolase activity [GO:0046573], monoacylglycerol lipase activity [GO:0047372], acetoxybutynylbithiophene deacetylase activity [GO:0047373], methylumbelliferyl-acetate deacetylase activity [GO:0047374], N-acetylgalactosaminoglycan deacetylase activity [GO:0047375], GO:0047377, acetylalkylglycerol acetylhydrolase activity [GO:0047378], 11-cis-retinyl-palmitate hydrolase activity [GO:0047520], 2-pyrone-4,6-dicarboxylate lactonase activity [GO:0047554], 3-oxoadipate enol-lactonase activity [GO:0047570], 4-methyloxaloacetate esterase activity [GO:0047583], GO:0047585, 6-acetylglucose deacetylase activity [GO:0047593], acetylsalicylate deacetylase activity [GO:0047610], actinomycin lactonase activity [GO:0047615], acylcarnitine hydrolase activity [GO:0047619], alpha-amino-acid esterase activity [GO:0047658], bis(2-ethylhexyl)phthalate esterase activity [GO:0047709], galactolipase activity [GO:0047714], cephalosporin-C deacetylase activity [GO:0047739], cetraxate benzylesterase activity [GO:0047741], chlorogenate hydrolase activity [GO:0047745], chlorophyllase activity [GO:0047746], GO:0047815, deoxylimonate A-ring-lactonase activity [GO:0047845], dihydrocoumarin hydrolase activity [GO:0047856], GO:0047908, hydroxybutyrate-dimer hydrolase activity [GO:0047989], GO:0050021, L-rhamnono-1,4-lactonase activity [GO:0050033], GO:0050055, orsellinate-depside hydrolase activity [GO:0050160], GO:0050181, phosphatidylinositol deacylase activity [GO:0050185], GO:0050253, sinapine esterase activity [GO:0050285], steroid-lactonase activity [GO:0050293], tannase activity [GO:0050318], triacetate-lactonase activity [GO:0050349], GO:0050357, GO:0050389, wax-ester hydrolase activity [GO:0050398], xylono-1,4-lactonase activity [GO:0050402], 1,4-lactonase activity [GO:0050490], cutinase activity [GO:0050525], poly(3-hydroxybutyrate) depolymerase activity [GO:0050526], poly(3-hydroxyoctanoate) depolymerase activity [GO:0050527], GO:0050528, polyneuridine-aldehyde esterase activity [GO:0050529], protein methylesterase activity [GO:0051723], brefeldin A esterase activity [GO:0052772], pectin acetylesterase activity [GO:0052793], GO:0052797, all-trans-retinyl-ester hydrolase, 11-cis retinol forming activity [GO:0052885], GO:0061463, diphthine methylesterase activity [GO:0061685], methyl indole-3-acetate esterase activity [GO:0080030], GO:0080031, methyl jasmonate esterase activity [GO:0080032], pheophytinase activity [GO:0080124], pimelyl-[acyl-carrier protein] methyl ester esterase activity [GO:0090499], heparan sulfate N-deacetylase activity [GO:0102140], GO:0102197, trans-permethrin hydrolase activity [GO:0102209], 2-oxo-3-(5-oxofuran-2-ylidene)propanoate lactonase activity [GO:0102355], mycophenolic acid acyl-glucuronide esterase activity [GO:0102390], aclacinomycin T methylesterase activity [GO:0102530], 4-sulfomuconolactone hydrolase activity [GO:0102998], GO:0106372, carboxylesterase activity [GO:0106435], GO:0120558, palmitoleyl hydrolase activity [GO:1990699] Also known as: carboxylate esterase activity, carboxylic esterase activity, hydrolase activity acting on ester bonds Sources: GOC:curators Definition: Catalysis of the hydrolysis of a carboxylic ester bond. Relationships: is a type of hydrolase activity, acting on ester bonds [GO:0016788]